{
  "gene_name": "HEAT repeat-containing protein 5B",
  "term_id": "GO:0005794",
  "gene": "UniProtKB:Q9P2D3",
  "term_label": "Golgi apparatus",
  "gene_symbol": "HEATR5B"
}